{
  "gene_symbol": "IL1A",
  "gene": "UniProtKB:P01583",
  "gene_name": "Interleukin-1 alpha",
  "term_label": "extracellular space",
  "term_id": "GO:0005615"
}